{
  "term_id": "GO:0001955",
  "gene_name": "Reversion-inducing cysteine-rich protein with Kazal motifs",
  "gene_symbol": "RECK",
  "term_label": "blood vessel maturation",
  "gene": "UniProtKB:O95980"
}